{
  "term_label": "kinetochore",
  "gene": "UniProtKB:O14965",
  "gene_symbol": "AURKA",
  "term_id": "GO:0000776",
  "gene_name": "Aurora kinase A"
}